{
  "term_id": "GO:0005793",
  "gene": "UniProtKB:P49257",
  "term_label": "endoplasmic reticulum-Golgi intermediate compartment",
  "gene_name": "Protein ERGIC-53",
  "gene_symbol": "LMAN1"
}